{
  "term_id": "GO:2001235",
  "gene": "UniProtKB:Q8WYH8",
  "gene_name": "Inhibitor of growth protein 5",
  "gene_symbol": "ING5",
  "term_label": "positive regulation of apoptotic signaling pathway"
}